{
  "term_id": "GO:0019829",
  "term_label": "ATPase-coupled monoatomic cation transmembrane transporter activity",
  "gene_symbol": "ATP13A5",
  "gene_name": "Probable cation-transporting ATPase 13A5",
  "gene": "UniProtKB:Q4VNC0"
}